metanephric juxtaglomerulus cell differentiation [GO:0072251] (biological process) Definition: The process in which relatively unspecialized cells acquire specialized structural and/or functional features that characterize the juxtaglomerulus cells of the metanephros as it progresses from its formation to the mature state. Relationships: is a type of juxtaglomerulus cell differentiation [GO:0072052]; is a type of cell differentiation involved in metanephros development [GO:0072202]; is part of metanephric juxtaglomerular apparatus development [GO:0072206] Sources: GOC:mtg_kidney_jan10